{
  "term_id": "GO:0005886",
  "term_label": "plasma membrane",
  "gene_symbol": "NEGR1",
  "gene": "UniProtKB:Q7Z3B1",
  "gene_name": "Neuronal growth regulator 1"
}